double membrane vesicle viral factory membrane [GO:0062242] (cellular component) Relationships: is a type of host cell cytoplasmic vesicle membrane [GO:0044162]; is part of GO:0039718 Subtypes: double membrane vesicle viral factory outer membrane [GO:0062243], double membrane vesicle viral factory inner membrane [GO:0062245] References: PMID:22440839 Definition: One of the two endoplasmic reticulum-derived lipid bilayer membranes that bound a double membrane vesicle viral factory. Also known as: membrane of double membrane vesicle viral factory